3alpha-hydroxy-ent-sandaracopimardiene 9-beta-monooxygenase activity [GO:0102597] (molecular function) Relationships: is a type of oxidoreductase activity, acting on paired donors, with incorporation or reduction of molecular oxygen, NAD(P)H as one donor, and incorporation of one atom of oxygen [GO:0016709] Sources: EC:1.14.14.122, GOC:pz Definition: Catalysis of the reaction: ent-sandaracopimaradien-3-beta-ol + NADPH + H+ + O2 = oryzalexin E + NADP + H2O.